{
  "term_label": "innate immune response",
  "term_id": "GO:0045087",
  "gene_symbol": "TRIM54",
  "gene": "UniProtKB:Q9BYV2",
  "gene_name": "Tripartite motif-containing protein 54"
}